{
  "gene": "UniProtKB:A6NMT0",
  "term_id": "UNKNOWN:0001",
  "term_label": "Unknown molecular function",
  "gene_name": "Homeobox protein DBX1",
  "gene_symbol": "DBX1"
}